glycerate 2-kinase activity [GO:0043798] (MF) Relationships: is a type of kinase activity [GO:0016301]; is a type of phosphotransferase activity, alcohol group as acceptor [GO:0016773] Definition: Catalysis of the reaction: D-glycerate + ATP = 2-phospho-D-glycerate + ADP. References: PMID:14413719 Sources: RHEA:27377 Also known as: glycerate kinase, D-glycerate 2-kinase activity